{
  "gene_name": "Phosphatidylinositol N-acetylglucosaminyltransferase subunit H",
  "term_id": "UNKNOWN:0001",
  "gene_symbol": "PIGH",
  "term_label": "Unknown molecular function",
  "gene": "UniProtKB:Q14442"
}